bacterial-type flagellum hook [GO:0009424] (CC) Definition: The portion of the bacterial-type flagellum that connects the filament to the basal body. Also known as: flagellar hook, flagellin-based flagellum hook Relationships: is_a GO:0110165; BFO_0000050 GO:0009288 References: PMID:10572114, PMID:12624192 Sources: GOC:cilia, GOC:mtg_sensu